{
  "term_label": "Unknown cellular component",
  "term_id": "UNKNOWN:0003",
  "gene": "UniProtKB:Q9H2I8",
  "gene_name": "Leucine-rich melanocyte differentiation-associated protein",
  "gene_symbol": "LRMDA"
}